{
  "term_label": "innate immune response",
  "gene_name": "Mucosa-associated lymphoid tissue lymphoma translocation protein 1",
  "gene": "UniProtKB:Q9UDY8",
  "term_id": "GO:0045087",
  "gene_symbol": "MALT1"
}